{
  "gene_symbol": "TULP1",
  "gene": "UniProtKB:O00294",
  "term_id": "GO:0005929",
  "gene_name": "Tubby-related protein 1",
  "term_label": "cilium"
}